{
  "gene": "UniProtKB:Q86Y29",
  "term_label": "Unknown cellular component",
  "gene_name": "B melanoma antigen 3",
  "term_id": "UNKNOWN:0003",
  "gene_symbol": "BAGE3"
}